{
  "gene": "UniProtKB:B3EWF7",
  "gene_name": "Laforin, isoform 9",
  "gene_symbol": "EPM2A",
  "term_id": "UNKNOWN:0003",
  "term_label": "Unknown cellular component"
}